{
  "term_label": "plasma membrane",
  "gene": "UniProtKB:P61764",
  "term_id": "GO:0005886",
  "gene_symbol": "STXBP1",
  "gene_name": "Syntaxin-binding protein 1"
}